{
  "gene_symbol": "IAPP",
  "term_label": "Unknown molecular function",
  "term_id": "UNKNOWN:0001",
  "gene_name": "Islet amyloid polypeptide",
  "gene": "UniProtKB:P10997"
}